{
  "gene_symbol": "KLHL14",
  "gene_name": "Kelch-like protein 14",
  "term_id": "GO:0043005",
  "gene": "UniProtKB:Q9P2G3",
  "term_label": "neuron projection"
}